{
  "gene_symbol": "CSNK1D",
  "gene_name": "Casein kinase I isoform delta",
  "term_label": "spindle microtubule",
  "gene": "UniProtKB:P48730",
  "term_id": "GO:0005876"
}